{
  "term_label": "positive regulation of canonical NF-kappaB signal transduction",
  "term_id": "GO:0043123",
  "gene": "UniProtKB:O15111",
  "gene_name": "Inhibitor of nuclear factor kappa-B kinase subunit alpha",
  "gene_symbol": "CHUK"
}